{
  "gene": "UniProtKB:Q58FF6",
  "term_label": "unfolded protein binding",
  "gene_name": "Putative heat shock protein HSP 90-beta 4",
  "gene_symbol": "HSP90AB4P",
  "term_id": "GO:0051082"
}